{
  "term_label": "mitochondrion",
  "gene": "UniProtKB:P82663",
  "term_id": "GO:0005739",
  "gene_symbol": "MRPS25",
  "gene_name": "Small ribosomal subunit protein mS25"
}